GAF domain binding [GO:0036004] (molecular function) Sources: GOC:yaf, InterPro:IPR003018 Definition: Binding to a GAF protein domain. Relationships: is a type of protein domain specific binding [GO:0019904]